DBIRD complex [GO:0044609] (cellular component) Relationships: is_a GO:0140535 References: PMID:22446626 Sources: GOC:sp Definition: A protein complex that associates with mRNP particles and RNA polymerase II and is proposed to integrate transcript elongation with the regulation of alternative splicing. In humans it is composed of the proteins KIAA1967/DBC1 and ZNF326/ZIRD.